positive regulation of myelination [GO:0031643] (biological process) Also known as: up regulation of myelination, up-regulation of myelination, upregulation of myelination, activation of myelination, stimulation of myelination Relationships: is a type of regulation of myelination [GO:0031641]; is a type of GO:0031646; is a type of positive regulation of cellular process [GO:0048522]; positively regulates myelination [GO:0042552] Sources: GOC:mah Definition: Any process that activates or increases the frequency, rate or extent of the formation of a myelin sheath around nerve axons.